{
  "gene_symbol": "STX1B",
  "term_id": "GO:0048278",
  "term_label": "vesicle docking",
  "gene_name": "Syntaxin-1B",
  "gene": "UniProtKB:P61266"
}